lysine biosynthetic process [GO:0009085] (biological process) Definition: The chemical reactions and pathways resulting in the formation of lysine, 2,6-diaminohexanoic acid. Sources: GOC:go_curators Also known as: lysine anabolism, lysine biosynthesis, lysine formation, lysine synthesis Relationships: is a type of lysine metabolic process [GO:0006553]; is a type of GO:0009067 Subtypes: lysine biosynthetic process via diaminopimelate [GO:0009089], lysine biosynthetic process via aminoadipic acid [GO:0019878]